{
  "gene_name": "Cannabinoid receptor 1",
  "term_id": "GO:0007189",
  "gene_symbol": "CNR1",
  "gene": "UniProtKB:P21554",
  "term_label": "adenylate cyclase-activating G protein-coupled receptor signaling pathway"
}